{
  "term_id": "GO:0051427",
  "gene": "UniProtKB:P01160",
  "term_label": "hormone receptor binding",
  "gene_name": "Natriuretic peptides A",
  "gene_symbol": "NPPA"
}